{
  "term_label": "receptor antagonist activity",
  "term_id": "GO:0048019",
  "gene_symbol": "MTRNR2L13",
  "gene_name": "Humanin-like 13",
  "gene": "UniProtKB:S4R3P1"
}